{
  "term_id": "GO:0005886",
  "gene": "UniProtKB:O14798",
  "gene_symbol": "TNFRSF10C",
  "term_label": "plasma membrane",
  "gene_name": "Tumor necrosis factor receptor superfamily member 10C"
}